{
  "gene_name": "Semaphorin-6C",
  "term_label": "neural crest cell migration",
  "gene": "UniProtKB:Q9H3T2",
  "gene_symbol": "SEMA6C",
  "term_id": "GO:0001755"
}